pyrimidine ribonucleoside triphosphate biosynthetic process [GO:0009209] (biological process) Relationships: is a type of GO:0009148; is a type of GO:0009201; is a type of GO:0009208 Sources: GOC:go_curators, ISBN:0198506732 Definition: The chemical reactions and pathways resulting in the formation of pyrimidine ribonucleoside triphosphate, a compound consisting of a pyrimidine base linked to a ribose sugar esterified with triphosphate on the sugar. Also known as: pyrimidine ribonucleoside triphosphate anabolism, pyrimidine ribonucleoside triphosphate biosynthesis, pyrimidine ribonucleoside triphosphate formation, pyrimidine ribonucleoside triphosphate synthesis Subtypes: GO:0006228, TTP biosynthetic process [GO:0006234], CTP biosynthetic process [GO:0006241]